cell elongation involved in imaginal disc-derived wing morphogenesis [GO:0090254] (biological process) Definition: The process in which a cell elongates and contributes to imaginal disc-derived wing morphogenesis. Sources: GOC:ascb_2009, GOC:dph, GOC:tb Relationships: is a type of unidimensional cell growth [GO:0009826]; is a type of GO:0009886; is part of imaginal disc-derived wing morphogenesis [GO:0007476]